negative regulation of miRNA transcription [GO:1902894] (BP) References: PMID:24699545 Sources: GOC:TermGenie, GOC:dph, GOC:kmv, GO_REF:0000058 Relationships: is a type of negative regulation of DNA-templated transcription [GO:0045892]; is a type of GO:1902893; is_a negative regulation of miRNA metabolic process [GO:2000629]; negatively regulates GO:0061614 Also known as: down regulation of pri-miRNA transcription from RNA polymerase II promoter, down-regulation of pri-miRNA transcription from RNA polymerase II promoter, downregulation of pri-miRNA transcription from RNA polymerase II promoter, negative regulation of miRNA gene transcription, negative regulation of microRNA gene transcription, negative regulation of pri-miRNA transcription by RNA polymerase II, negative regulation of pri-miRNA transcription from RNA polymerase II promoter, negative regulation of primary miRNA gene transcription, inhibition of pri-miRNA transcription from RNA polymerase II promoter Definition: Any process that stops, prevents or reduces the frequency, rate or extent of microRNA (miRNA) gene transcription.